regulation of protein localization to early endosome [GO:1902965] (biological process) Subtypes: GO:1902966 Also known as: regulation of protein localisation in early endosome, regulation of protein localisation to early endosome, regulation of protein localization in early endosome Definition: Any process that modulates the frequency, rate or extent of protein localization to early endosome. References: PMID:22621900 Sources: GOC:TermGenie, GOC:sjp, GO_REF:0000058 Relationships: is a type of GO:1905666; regulates protein localization to early endosome [GO:1902946]